{
  "gene_symbol": "FSTL3",
  "term_id": "GO:0048185",
  "term_label": "activin binding",
  "gene_name": "Follistatin-related protein 3",
  "gene": "UniProtKB:O95633"
}